acylglycerol homeostasis [GO:0055090] (biological process) Relationships: is a type of lipid homeostasis [GO:0055088] Also known as: glyceride homeostasis Subtypes: triglyceride homeostasis [GO:0070328] Definition: Any process involved in the maintenance of an internal steady state of acylglycerol within an organism or cell. Sources: GOC:BHF, GOC:rl